{
  "gene_name": "Zinc finger protein 561",
  "gene_symbol": "ZNF561",
  "gene": "UniProtKB:Q8N587",
  "term_label": "regulation of transcription by RNA polymerase II",
  "term_id": "GO:0006357"
}